{
  "gene_symbol": "KRTAP10-11",
  "gene": "UniProtKB:P60412",
  "gene_name": "Keratin-associated protein 10-11",
  "term_id": "UNKNOWN:0001",
  "term_label": "Unknown molecular function"
}